{
  "gene": "UniProtKB:Q92637",
  "gene_symbol": "FCGR1BP",
  "gene_name": "Putative high affinity immunoglobulin gamma Fc receptor IB",
  "term_label": "positive regulation of tumor necrosis factor production",
  "term_id": "GO:0032760"
}